glutathione derivative catabolic process [GO:1901686] (biological process) Subtypes: GO:0046207 Sources: GOC:TermGenie, GOC:pr Also known as: glutathione derivative breakdown, glutathione derivative catabolism, glutathione derivative degradation Relationships: is a type of sulfur compound catabolic process [GO:0044273] Definition: The chemical reactions and pathways resulting in the breakdown of glutathione derivative.